{
  "term_label": "Unknown cellular component",
  "gene_name": "PWWP domain-containing DNA repair factor 4",
  "term_id": "UNKNOWN:0003",
  "gene_symbol": "PWWP4",
  "gene": "UniProtKB:A0A494C071"
}